glutamyl-tRNA aminoacylation [GO:0006424] (biological process) Definition: The process of coupling glutamate to glutamyl-tRNA, catalyzed by glutamyl-tRNA synthetase. The glutamyl-tRNA synthetase is a class-I synthetase. The activated amino acid is transferred to the 2'-OH group of a glutamic acid-accetping tRNA. The 2'-O-aminoacyl-tRNA will ultimately migrate to the 3' position via transesterification. Sources: GOC:mcc, ISBN:0716730510 Relationships: is a type of tRNA aminoacylation for protein translation [GO:0006418] Subtypes: mitochondrial glutamyl-tRNA aminoacylation [GO:0070149]